{
  "gene_name": "Cystin-1",
  "gene": "UniProtKB:Q717R9",
  "term_label": "Unknown cellular component",
  "gene_symbol": "CYS1",
  "term_id": "UNKNOWN:0003"
}